{
  "term_id": "GO:0005886",
  "gene": "UniProtKB:Q14568",
  "gene_name": "Heat shock protein HSP 90-alpha A2",
  "gene_symbol": "HSP90AA2P",
  "term_label": "plasma membrane"
}